masculinization of hermaphrodite soma [GO:0042003] (BP) Definition: Promotion of male sex and sexual phenotypes in the hermaphroditic nematode soma. An example of this is found in Caenorhabditis elegans. Sources: GOC:ems Relationships: is a type of hermaphrodite somatic sex determination [GO:0042001]